{
  "term_id": "GO:0000139",
  "gene": "UniProtKB:Q9H3P7",
  "gene_symbol": "ACBD3",
  "term_label": "Golgi membrane",
  "gene_name": "Golgi resident protein GCP60"
}